pentadec-1-ene biosynthetic process [GO:1900873] (biological process) Also known as: pentadec-1-ene anabolism, pentadec-1-ene biosynthesis, pentadec-1-ene formation, pentadec-1-ene synthesis Sources: GOC:TermGenie, GOC:mengo_curators Relationships: is a type of alkene biosynthetic process [GO:0043450] Definition: The chemical reactions and pathways resulting in the formation of pentadec-1-ene.